{
  "gene_name": "Disks large homolog 4",
  "term_id": "GO:0098609",
  "gene": "UniProtKB:P78352",
  "term_label": "cell-cell adhesion",
  "gene_symbol": "DLG4"
}